{
  "term_id": "GO:1990481",
  "gene_name": "H_ACA ribonucleoprotein complex subunit DKC1",
  "gene": "UniProtKB:O60832",
  "term_label": "mRNA pseudouridine synthesis",
  "gene_symbol": "DKC1"
}